{
  "term_label": "positive regulation of vasoconstriction",
  "gene_name": "Vasopressin-neurophysin 2-copeptin",
  "gene_symbol": "AVP",
  "gene": "UniProtKB:P01185",
  "term_id": "GO:0045907"
}